{
  "term_label": "chromatin binding",
  "term_id": "GO:0003682",
  "gene": "UniProtKB:Q8N7H5",
  "gene_name": "RNA polymerase II-associated factor 1 homolog",
  "gene_symbol": "PAF1"
}